zygotic specification of dorsal/ventral axis [GO:0007352] (biological process) Definition: The specification of the dorsal/ventral axis of the embryo, through the products of genes expressed in the zygote. Sources: GOC:bf Also known as: zygotic determination of dorsal-ventral axis, zygotic determination of dorsal/ventral axis, zygotic determination of dorsoventral axis Relationships: is a type of embryonic axis specification [GO:0000578]; is a type of dorsal/ventral axis specification [GO:0009950]